{
  "gene": "UniProtKB:Q13123",
  "term_id": "UNKNOWN:0001",
  "term_label": "Unknown molecular function",
  "gene_symbol": "IK",
  "gene_name": "Protein Red"
}